{
  "term_label": "sodium:potassium-exchanging ATPase complex",
  "gene": "UniProtKB:P54709",
  "term_id": "GO:0005890",
  "gene_symbol": "ATP1B3",
  "gene_name": "Sodium_potassium-transporting ATPase subunit beta-3"
}